{
  "gene": "UniProtKB:Q8WU17",
  "term_label": "ubiquitin protein ligase activity",
  "gene_name": "E3 ubiquitin-protein ligase RNF139",
  "gene_symbol": "RNF139",
  "term_id": "GO:0061630"
}